{
  "gene_name": "AP-1 complex subunit mu-1",
  "term_label": "trans-Golgi network",
  "gene_symbol": "AP1M1",
  "gene": "UniProtKB:Q9BXS5",
  "term_id": "GO:0005802"
}